{
  "gene_symbol": "DCP1B",
  "gene_name": "mRNA-decapping enzyme 1B",
  "term_label": "deadenylation-dependent decapping of nuclear-transcribed mRNA",
  "term_id": "GO:0000290",
  "gene": "UniProtKB:Q8IZD4"
}